{
  "gene": "UniProtKB:Q12904",
  "term_label": "Unknown cellular component",
  "gene_symbol": "AIMP1",
  "term_id": "UNKNOWN:0003",
  "gene_name": "Aminoacyl tRNA synthase complex-interacting multifunctional protein 1"
}